quinolinate biosynthetic process [GO:0019805] (BP) Relationships: is a type of dicarboxylic acid biosynthetic process [GO:0043650]; is a type of quinolinate metabolic process [GO:0046874]; is a type of pyridine-containing compound biosynthetic process [GO:0072525] Also known as: quinolinate anabolism, quinolinate biosynthesis, quinolinate formation, quinolinate synthesis Definition: The chemical reactions and pathways resulting in the formation of quinolinate, the anion of quinolinic acid, also known as 2,3-pyridinedicarboxylic acid. Regulation: regulated by regulation of quinolinate biosynthetic process [GO:1904984]; RO_0002212 by negative regulation of quinolinate biosynthetic process [GO:1904985]; positively regulated by positive regulation of quinolinate biosynthetic process [GO:1904986] Sources: GOC:ai